{
  "term_label": "positive regulation of DNA-templated transcription",
  "term_id": "GO:0045893",
  "gene": "UniProtKB:Q9UJW9",
  "gene_symbol": "SERTAD3",
  "gene_name": "SERTA domain-containing protein 3"
}